{
  "term_id": "UNKNOWN:0001",
  "gene_symbol": "CAPS2",
  "gene": "UniProtKB:Q9BXY5",
  "gene_name": "Calcyphosin-2",
  "term_label": "Unknown molecular function"
}